ribosylpyrimidine nucleosidase activity [GO:0050263] (molecular function) Sources: EC:3.2.2.8, MetaCyc:RIBOSYLPYRIMIDINE-NUCLEOSIDASE-RXN Also known as: nucleoside ribohydrolase activity, N-ribosylpyrimidine nucleosidase activity, N-ribosylpyrimidine ribohydrolase activity, RihB, YeiK, pyrimidine nucleosidase activity, pyrimidine-nucleoside ribohydrolase activity Definition: Catalysis of the reaction: an N-D-ribosylpyrimidine + H2O = D-ribose + a pyrimidine. Subtypes: uridine nucleosidase activity [GO:0045437] Relationships: is a type of hydrolase activity, hydrolyzing N-glycosyl compounds [GO:0016799]